{
  "gene_name": "Peptidyl-prolyl cis-trans isomerase FKBP9",
  "term_label": "peptidyl-prolyl cis-trans isomerase activity",
  "gene": "UniProtKB:O95302",
  "term_id": "GO:0003755",
  "gene_symbol": "FKBP9"
}